perinuclear endoplasmic reticulum lumen [GO:0099020] (cellular component) Sources: GOC:dos, GOC:vw Relationships: is a type of endoplasmic reticulum lumen [GO:0005788]; is part of perinuclear endoplasmic reticulum [GO:0097038] Definition: The volume enclosed by the membranes of the perinuclear endoplasmic reticulum.